{
  "term_id": "GO:0000978",
  "gene_name": "Homeobox protein Hox-C9",
  "term_label": "RNA polymerase II cis-regulatory region sequence-specific DNA binding",
  "gene": "UniProtKB:P31274",
  "gene_symbol": "HOXC9"
}